{
  "gene_symbol": "PCBP2",
  "term_id": "GO:0003729",
  "gene": "UniProtKB:Q15366",
  "term_label": "mRNA binding",
  "gene_name": "Poly(rC)-binding protein 2"
}